{
  "gene": "UniProtKB:Q9BQQ3",
  "gene_name": "Golgi reassembly-stacking protein 1",
  "term_label": "Golgi apparatus",
  "gene_symbol": "GORASP1",
  "term_id": "GO:0005794"
}